negative regulation of phospholipase C-activating dopamine receptor signaling pathway [GO:0060162] (biological process) Also known as: negative regulation of dopamine receptor, phospholipase C activating pathway, negative regulation of phospholipase C-activating dopamine receptor signalling pathway References: PMID:15016423 Sources: GOC:dph, GOC:tb Relationships: is_a GO:0060160; is a type of negative regulation of phospholipase C-activating G protein-coupled receptor signaling pathway [GO:1900737]; negatively regulates phospholipase C-activating dopamine receptor signaling pathway [GO:0060158] Definition: Any process that stops, prevents, or reduces the frequency, rate or extent of the dopamine receptor, phospholipase C activating pathway.